{
  "gene_symbol": "RYR3",
  "gene": "UniProtKB:Q15413",
  "term_id": "GO:0030018",
  "term_label": "Z disc",
  "gene_name": "Ryanodine receptor 3"
}